alphaPDGFR-SHP-2 complex [GO:0070718] (cellular component) Also known as: PDGFRA-SHP-2 complex, PDGF stimulated References: PMID:8943348 Sources: GOC:mah Relationships: is a type of plasma membrane protein complex [GO:0098797] Definition: A protein complex that contains the platelet-derived growth factor alpha receptor (alphaPDGFR; PDGFRA) and the adaptor protein SHP-2, and is involved signaling via the PDGFR signaling pathway.